{
  "gene": "UniProtKB:P24386",
  "gene_name": "Rab proteins geranylgeranyltransferase component A 1",
  "term_label": "Unknown molecular function",
  "term_id": "UNKNOWN:0001",
  "gene_symbol": "CHM"
}